{
  "gene": "UniProtKB:Q96BR9",
  "term_id": "GO:0000978",
  "gene_symbol": "ZBTB8A",
  "term_label": "RNA polymerase II cis-regulatory region sequence-specific DNA binding",
  "gene_name": "Zinc finger and BTB domain-containing protein 8A"
}